{
  "gene": "UniProtKB:P54756",
  "term_label": "plasma membrane",
  "gene_symbol": "EPHA5",
  "term_id": "GO:0005886",
  "gene_name": "Ephrin type-A receptor 5"
}